negative regulation of inosine transport [GO:0035343] (biological process) Relationships: is a type of negative regulation of purine nucleoside transport [GO:0032247]; is a type of regulation of inosine transport [GO:0035341]; negatively regulates inosine transport [GO:0035340] Also known as: negative regulation of hypoxanthine riboside transport Sources: GOC:bf Definition: Any process that stops, prevents, or reduces the frequency, rate or extent of the directed movement of inosine into, out of or within a cell, or between cells, by means of some agent such as a transporter or pore.